growth hormone secretagogue receptor activity [GO:0001616] (molecular function) References: PMID:17983853 Sources: GOC:mah Definition: Combining with ghrelin to initiate a change in cell activity. Relationships: is_a GO:0004930 Also known as: ghrelin receptor activity